{
  "gene_symbol": "PTPA",
  "term_label": "mitotic spindle organization",
  "term_id": "GO:0007052",
  "gene": "UniProtKB:Q15257",
  "gene_name": "Serine_threonine-protein phosphatase 2A activator"
}